{
  "gene_symbol": "DEPDC5",
  "term_id": "GO:1904262",
  "gene_name": "GATOR complex protein DEPDC5",
  "term_label": "negative regulation of TORC1 signaling",
  "gene": "UniProtKB:O75140"
}